{
  "term_id": "GO:0005737",
  "term_label": "cytoplasm",
  "gene_name": "Tripartite motif-containing protein 64C",
  "gene_symbol": "TRIM64C",
  "gene": "UniProtKB:A6NLI5"
}